{
  "term_id": "GO:0004930",
  "gene_symbol": "DRD5",
  "gene_name": "D(1B) dopamine receptor",
  "term_label": "G protein-coupled receptor activity",
  "gene": "UniProtKB:P21918"
}